monopolin complex [GO:0033551] (cellular component) Definition: A protein complex required for clamping microtubule binding sites, ensuring orientation of sister kinetochores to the same pole (mono-orientation) during meiosis I. In the yeast S. cerevisiae this complex consists of Csm1p, Lrs4p, Hrr25p and Mam1p; in S. pombe Psc1 and Mde4 have been identified as subunits. References: PMID:17627824 Sources: GOC:mah, GOC:rb Also known as: Pcs1/Mde4 complex, monopolin subcomplex Csm1/Lrs4 Relationships: is a type of GO:0032991; is part of kinetochore [GO:0000776]